{
  "term_id": "GO:0005886",
  "term_label": "plasma membrane",
  "gene_name": "Glutamate receptor 4",
  "gene_symbol": "GRIA4",
  "gene": "UniProtKB:P48058"
}